{
  "gene_symbol": "DENND10P1",
  "term_id": "GO:0005085",
  "gene": "UniProtKB:Q6NSW5",
  "term_label": "guanyl-nucleotide exchange factor activity",
  "gene_name": "Putative DENN domain-containing protein 10 B"
}